toxin metabolic process [GO:0009404] (biological process) Sources: GOC:cab2 Subtypes: toxin biosynthetic process [GO:0009403], GO:0009407, insecticide metabolic process [GO:0017143], bacteriocin immunity [GO:0030153], GO:0043385, sterigmatocystin metabolic process [GO:0045460], bacteriocin metabolic process [GO:0046224], phytoalexin metabolic process [GO:0052314] Relationships: is_a secondary metabolic process [GO:0019748] Definition: The chemical reactions and pathways involving a toxin, a poisonous compound (typically a protein) that is produced by cells or organisms and that can cause disease when introduced into the body or tissues of an organism. Also known as: toxin metabolism